{
  "gene": "UniProtKB:Q6ZQN7",
  "gene_symbol": "SLCO4C1",
  "term_label": "Unknown molecular function",
  "term_id": "UNKNOWN:0001",
  "gene_name": "Solute carrier organic anion transporter family member 4C1"
}